apicoplast membrane [GO:0160211] (cellular component) Relationships: is_a plastid membrane [GO:0042170]; is part of GO:0020011 References: PMID:20124342, PMID:38865262 Definition: Any of the lipid bilayers that surround an apicoplast and form the apicoplast envelope.